{
  "gene_symbol": "MYOC",
  "term_id": "GO:0005794",
  "term_label": "Golgi apparatus",
  "gene_name": "Myocilin",
  "gene": "UniProtKB:Q99972"
}